{
  "gene_symbol": "BIRC2",
  "gene": "UniProtKB:Q13490",
  "term_id": "GO:0031398",
  "term_label": "positive regulation of protein ubiquitination",
  "gene_name": "Baculoviral IAP repeat-containing protein 2"
}